{
  "gene": "UniProtKB:Q9BXQ6",
  "term_id": "UNKNOWN:0003",
  "term_label": "Unknown cellular component",
  "gene_symbol": "TMEM121B",
  "gene_name": "Transmembrane protein 121B"
}